{
  "gene_name": "Otogelin",
  "gene_symbol": "OTOG",
  "term_id": "GO:0031012",
  "gene": "UniProtKB:Q6ZRI0",
  "term_label": "extracellular matrix"
}